transmission of nerve impulse [GO:0019226] (biological process) Definition: The neurological system process in which a signal is transmitted through the nervous system by a combination of action potential propagation and synaptic transmission. Relationships: is_a GO:0050877; is part of GO:0007154; has part GO:0001508; has part chemical synaptic transmission [GO:0007268] Regulation: regulated by regulation of transmission of nerve impulse [GO:0051969]; negatively regulated by negative regulation of transmission of nerve impulse [GO:0051970]; positively regulated by positive regulation of transmission of nerve impulse [GO:0051971] Sources: GOC:curators, ISBN:0815316194 Also known as: conduction of nerve impulse, signal transmission along a neuron